{
  "gene": "UniProtKB:P17813",
  "gene_symbol": "ENG",
  "gene_name": "Endoglin",
  "term_id": "GO:0001570",
  "term_label": "vasculogenesis"
}